{
  "term_label": "K63-linked deubiquitinase activity",
  "gene_symbol": "STAMBP",
  "gene": "UniProtKB:O95630",
  "gene_name": "STAM-binding protein",
  "term_id": "GO:0061578"
}